protein localization to postsynaptic membrane [GO:1903539] (biological process) References: PMID:9753322 Sources: GOC:TermGenie, GOC:kmv, GO_REF:0000087 Subtypes: neurotransmitter receptor transport to postsynaptic membrane [GO:0098969], protein localization to postsynaptic specialization membrane [GO:0099633] Relationships: is a type of GO:0062237; is a type of protein localization to membrane [GO:0072657]; is a type of GO:1990778 Also known as: protein localisation in postsynaptic membrane, protein localisation to postsynaptic membrane, protein localization in postsynaptic membrane Definition: A process in which a protein is transported to, or maintained in, a location within a postsynaptic membrane.